L-type voltage-gated calcium channel complex [GO:1990454] (cellular component) Definition: A type of voltage-dependent calcium channel responsible for excitation-contraction coupling of skeletal, smooth, and cardiac muscle. 'L' stands for 'long-lasting' referring to the length of activation. References: PMID:12946355 Sources: GOC:ame Relationships: is a type of voltage-gated calcium channel complex [GO:0005891]; is part of T-tubule [GO:0030315] Note: Examples of this are CACNA1S, CACNA2D1, CACNB1, CACNG1 in rabbit (UniProt symbol P07293, P13806, P19517 and P19518) in PMID:12946355 (inferred from direct assay). Also known as: cardiac muscle L-type voltage-gated calcium channel complex, skeletal muscle L-type voltage-gated calcium channel complex